inosine metabolic process [GO:0046102] (biological process) Sources: GOC:go_curators Definition: The chemical reactions and pathways involving inosine, hypoxanthine riboside, a nucleoside found free but not in combination in nucleic acids except in the anticodons of some tRNAs. Also known as: inosine metabolism Subtypes: inosine catabolic process [GO:0006148], GO:0046103 Relationships: is_a purine ribonucleoside metabolic process [GO:0046128]